{
  "term_label": "Unknown molecular function",
  "gene_symbol": "FYB2",
  "gene_name": "FYN-binding protein 2",
  "gene": "UniProtKB:Q5VWT5",
  "term_id": "UNKNOWN:0001"
}